{
  "term_label": "branched-chain alpha-ketoacid dehydrogenase complex",
  "gene_symbol": "DBT",
  "gene": "UniProtKB:P11182",
  "gene_name": "Lipoamide acyltransferase component of branched-chain alpha-keto acid dehydrogenase complex, mitochondrial",
  "term_id": "GO:0160157"
}